{
  "term_id": "GO:0043473",
  "term_label": "pigmentation",
  "gene_symbol": "TYR",
  "gene": "UniProtKB:P14679",
  "gene_name": "Tyrosinase"
}